{
  "gene_symbol": "SPMIP8",
  "gene": "UniProtKB:Q6URK8",
  "gene_name": "Testis, prostate and placenta-expressed protein",
  "term_id": "GO:0160111",
  "term_label": "axonemal A tubule inner sheath"
}